{
  "term_id": "UNKNOWN:0001",
  "gene_name": "Putative transcriptional regulator encoded by LINC00473",
  "gene_symbol": "LINC00473",
  "term_label": "Unknown molecular function",
  "gene": "UniProtKB:A8K010"
}